{
  "term_id": "UNKNOWN:0001",
  "term_label": "Unknown molecular function",
  "gene_name": "Transmembrane protein 92",
  "gene": "UniProtKB:Q6UXU6",
  "gene_symbol": "TMEM92"
}